seed trichome maturation [GO:0090380] (biological process) Note: These processes continue to 60 DPA in Gossypium spp. Relationships: is a type of developmental process involved in reproduction [GO:0003006]; is a type of cellular process involved in reproduction in multicellular organism [GO:0022412]; is a type of cell maturation [GO:0048469]; is part of GO:0090376 Definition: A developmental process, independent of morphogenetic (shape) change, that is required for a seed trichome to attain its fully functional state. Sources: GOC:tb